{
  "gene_symbol": "RNF8",
  "gene_name": "E3 ubiquitin-protein ligase RNF8",
  "term_id": "GO:0042393",
  "gene": "UniProtKB:O76064",
  "term_label": "histone binding"
}